{
  "term_id": "UNKNOWN:0002",
  "gene": "UniProtKB:A4IF30",
  "term_label": "Unknown biological process",
  "gene_symbol": "SLC35F4",
  "gene_name": "Solute carrier family 35 member F4"
}